{
  "term_label": "cytoplasm",
  "term_id": "GO:0005737",
  "gene_name": "Putative oncomodulin-2",
  "gene": "UniProtKB:P0CE71",
  "gene_symbol": "OCM2"
}